positive regulation by virus of viral protein levels in host cell [GO:0046726] (biological process) Sources: GOC:ai Relationships: is_a regulation by virus of viral protein levels in host cell [GO:0046719]; is a type of positive regulation of viral process [GO:0048524] Also known as: positive regulation of viral protein levels, up regulation of viral protein levels in host cell, up-regulation of viral protein levels in host cell, upregulation of viral protein levels in host cell, activation of viral protein levels in host cell, stimulation of viral protein levels in host cell Definition: Any process where the infecting virus increases the levels of viral proteins in a cell.